{
  "gene": "UniProtKB:Q9C005",
  "gene_symbol": "DPY30",
  "term_label": "Unknown cellular component",
  "gene_name": "Protein dpy-30 homolog",
  "term_id": "UNKNOWN:0003"
}